{
  "gene": "UniProtKB:Q9H790",
  "gene_symbol": "EXO5",
  "gene_name": "Exonuclease V",
  "term_label": "nucleus",
  "term_id": "GO:0005634"
}